carboxypeptidase activity [GO:0004180] (molecular function) Relationships: is a type of exopeptidase activity [GO:0008238] Subtypes: metallocarboxypeptidase activity [GO:0004181], serine-type carboxypeptidase activity [GO:0004185], cysteine-type carboxypeptidase activity [GO:0016807], GO:0106415 Definition: Catalysis of the hydrolysis of a single C-terminal amino acid residue from a polypeptide chain. Sources: https://www.ebi.ac.uk/merops/about/glossary.shtml#CARBOXYPEPTIDASE